{
  "gene_name": "DENN domain-containing protein 1C",
  "gene": "UniProtKB:Q8IV53",
  "term_label": "cytosol",
  "gene_symbol": "DENND1C",
  "term_id": "GO:0005829"
}